{
  "gene_symbol": "FBXL12",
  "gene": "UniProtKB:Q9NXK8",
  "term_id": "GO:0019005",
  "term_label": "SCF ubiquitin ligase complex",
  "gene_name": "F-box_LRR-repeat protein 12"
}